{
  "term_id": "GO:0005829",
  "term_label": "cytosol",
  "gene": "UniProtKB:D6RCP7",
  "gene_name": "Ubiquitin carboxyl-terminal hydrolase 17-like protein 19",
  "gene_symbol": "USP17L19"
}